{
  "term_id": "GO:0042632",
  "term_label": "cholesterol homeostasis",
  "gene_symbol": "LDAH",
  "gene": "UniProtKB:Q9H6V9",
  "gene_name": "Lipid droplet-associated hydrolase"
}